{
  "term_id": "GO:0006289",
  "gene_name": "Fanconi anemia group C protein",
  "gene_symbol": "FANCC",
  "term_label": "nucleotide-excision repair",
  "gene": "UniProtKB:Q00597"
}